{
  "gene": "UniProtKB:P42696",
  "term_id": "GO:0003723",
  "term_label": "RNA binding",
  "gene_symbol": "RBM34",
  "gene_name": "RNA-binding protein 34"
}